{
  "gene_name": "Zinc finger protein 345",
  "term_id": "GO:0005634",
  "gene_symbol": "ZNF345",
  "gene": "UniProtKB:Q14585",
  "term_label": "nucleus"
}